{
  "gene": "UniProtKB:P62318",
  "term_label": "RNA binding",
  "term_id": "GO:0003723",
  "gene_symbol": "SNRPD3",
  "gene_name": "Small nuclear ribonucleoprotein Sm D3"
}